{
  "gene_name": "Solute carrier family 12 member 5",
  "gene": "UniProtKB:Q9H2X9",
  "gene_symbol": "SLC12A5",
  "term_id": "GO:0007268",
  "term_label": "chemical synaptic transmission"
}